{
  "gene": "UniProtKB:Q9NRZ9",
  "term_label": "pericentric heterochromatin",
  "gene_symbol": "HELLS",
  "gene_name": "Lymphoid-specific helicase",
  "term_id": "GO:0005721"
}